L-asparagine metabolic process [GO:0070982] (biological process) Also known as: L-asparagine metabolism Relationships: is a type of asparagine metabolic process [GO:0006528]; is a type of amide metabolic process [GO:0043603]; is a type of L-amino acid metabolic process [GO:0170033]; is_a proteinogenic amino acid metabolic process [GO:0170039] Subtypes: L-asparagine catabolic process [GO:0006530], L-asparagine biosynthetic process [GO:0070981] Definition: The chemical reactions and pathways involving L-asparagine, (2S)-2-amino-3-carbamoylpropanoic acid. Sources: GOC:mah